POU domain binding [GO:0070974] (molecular function) Relationships: is a type of protein domain specific binding [GO:0019904] Sources: GOC:mah, GOC:yaf, InterPro:IPR000327 Definition: Binding to a POU domain of a protein. The POU domain is a bipartite DNA binding domain composed of two subunits separated by a non-conserved region of 15-55 amino acids; it is found in several eukaryotic transcription factors.